{
  "term_label": "Unknown molecular function",
  "gene_name": "Glutathione hydrolase 6",
  "gene_symbol": "GGT6",
  "term_id": "UNKNOWN:0001",
  "gene": "UniProtKB:Q6P531"
}